{
  "term_id": "GO:0004623",
  "gene_symbol": "PLAAT4",
  "gene_name": "Phospholipase A and acyltransferase 4",
  "term_label": "phospholipase A2 activity",
  "gene": "UniProtKB:Q9UL19"
}